cellular bud neck contractile ring [GO:0000142] (CC) References: PMID:16009555 Sources: GOC:krc Definition: A contractile ring, i.e. a cytoskeletal structure composed of actin filaments and myosin, that forms beneath the plasma membrane at the mother-bud neck in mitotic cells that divide by budding in preparation for completing cytokinesis. An example of this structure is found in Saccharomyces cerevisiae. Relationships: is a type of mitotic actomyosin contractile ring [GO:0110085]; is part of cellular bud neck [GO:0005935] Also known as: neck ring